{
  "gene": "UniProtKB:Q9NWZ8",
  "term_id": "GO:0032797",
  "term_label": "SMN complex",
  "gene_name": "Gem-associated protein 8",
  "gene_symbol": "GEMIN8"
}